{
  "gene_name": "Mitochondrial carrier homolog 1",
  "term_id": "UNKNOWN:0001",
  "gene_symbol": "MTCH1",
  "gene": "UniProtKB:Q9NZJ7",
  "term_label": "Unknown molecular function"
}